oxidoreductase activity, acting on the CH-CH group of donors, iron-sulfur protein as acceptor [GO:0016636] (molecular function) Definition: Catalysis of an oxidation-reduction (redox) reaction in which a CH-CH group acts as a hydrogen or electron donor and reduces an iron-sulfur protein. Relationships: is a type of oxidoreductase activity, acting on the CH-CH group of donors [GO:0016627] Sources: EC:1.3.7.- Subtypes: benzoyl-CoA reductase activity [GO:0018522], 4-hydroxybenzoyl-CoA reductase activity [GO:0018525], 6-hydroxynicotinate reductase activity [GO:0047595], GO:0050617, GO:0050618, phytochromobilin:ferredoxin oxidoreductase activity [GO:0050619], phycocyanobilin:ferredoxin oxidoreductase activity [GO:0050620], GO:0051743 Also known as: oxidoreductase activity, acting on the CH-CH group of donors, iron-sulphur protein as acceptor